{
  "gene_name": "Histone-lysine N-methyltransferase SETD7",
  "gene_symbol": "SETD7",
  "term_label": "histone H3 methyltransferase activity",
  "gene": "UniProtKB:Q8WTS6",
  "term_id": "GO:0140938"
}